{
  "term_label": "Unknown biological process",
  "gene_symbol": "Q6ZSR9",
  "gene": "UniProtKB:Q6ZSR9",
  "gene_name": "Uncharacterized protein FLJ45252",
  "term_id": "UNKNOWN:0002"
}